(E)-caffeate-CoA ligase activity [GO:0106286] (molecular function) Relationships: is a type of GO:0016405 References: PMID:22649270 Sources: RHEA:36299 Definition: Catalysis of the reaction: (E)-caffeate + ATP + CoA = (E)-caffeoyl-CoA + AMP + diphosphate.